{
  "gene_symbol": "FHDC1",
  "term_id": "UNKNOWN:0001",
  "gene": "UniProtKB:Q9C0D6",
  "gene_name": "FH2 domain-containing protein 1",
  "term_label": "Unknown molecular function"
}